RNA catabolic process [GO:0006401] (biological process) Subtypes: RNA fragment catabolic process [GO:0000292], mitochondrial RNA catabolic process [GO:0000957], mRNA catabolic process [GO:0006402], miRNA catabolic process [GO:0010587], rRNA catabolic process [GO:0016075], GO:0016076, sno(s)RNA catabolic process [GO:0016077], tRNA decay [GO:0016078], GO:0034586, DNA replication, removal of RNA primer [GO:0043137], polyadenylation-dependent RNA catabolic process [GO:0043633], RNA surveillance [GO:0071025], CUT catabolic process [GO:0071034], GO:0110064, siRNA catabolic process [GO:0140746], pre-mRNA catabolic process [GO:1990261] Definition: The chemical reactions and pathways resulting in the breakdown of RNA, ribonucleic acid, one of the two main type of nucleic acid, consisting of a long, unbranched macromolecule formed from ribonucleotides joined in 3',5'-phosphodiester linkage. Relationships: is a type of RNA metabolic process [GO:0016070]; is a type of GO:0141188 Also known as: RNA breakdown, RNA catabolism, RNA degradation Sources: ISBN:0198506732 Regulation: RO_0002211 by GO:0043487; positively regulated by RNA destabilization [GO:0050779]; negatively regulated by negative regulation of RNA catabolic process [GO:1902369]